response to heat [GO:0009408] (biological process) Definition: Any process that results in a change in state or activity of a cell or an organism (in terms of movement, secretion, enzyme production, gene expression, etc.) as a result of a heat stimulus, a temperature stimulus above the optimal temperature for that organism. Also known as: response to heat shock Sources: GOC:lr Relationships: is a type of GO:0006950; is a type of response to temperature stimulus [GO:0009266] Subtypes: GO:0010286, GO:0034605, filamentous growth of a population of unicellular organisms in response to heat [GO:0036168]